{
  "gene": "UniProtKB:Q8N146",
  "term_label": "G protein-coupled receptor signaling pathway",
  "term_id": "GO:0007186",
  "gene_name": "Olfactory receptor 8H3",
  "gene_symbol": "OR8H3"
}